xyloglucan 4-glucosyltransferase activity [GO:0033826] (molecular function) Definition: Catalysis of the transfer of a beta-D-glucosyl residue from UDP-glucose on to a glucose residue in xyloglucan, forming a beta-1,4-D-glucosyl-D-glucose linkage. Also known as: UDP-glucose:xyloglucan 1,4-beta-D-glucosyltransferase activity, UDPglucose:xyloglucan 1,4-beta-D-glucosyltransferase activity, uridine diphosphoglucose-xyloglucan 4beta-glucosyltransferase activity, xyloglucan 4beta-D-glucosyltransferase activity, xyloglucan glucosyltransferase activity Relationships: is a type of GO:0046527 Sources: EC:2.4.1.168